protein-DNA complex assembly [GO:0065004] (biological process) Definition: The aggregation, arrangement and bonding together of proteins and DNA molecules to form a protein-DNA complex. Sources: GOC:jl Also known as: DNA-protein complex assembly Relationships: is a type of protein-containing complex assembly [GO:0065003]; is a type of GO:0071824 Subtypes: DNA recombinase assembly [GO:0000730], nucleotide-excision repair, preincision complex assembly [GO:0006294], nucleosome assembly [GO:0006334], protein-DNA ISRE complex assembly [GO:0035362], pre-replicative complex assembly [GO:0036388], transcription preinitiation complex assembly [GO:0070897], DNA replication preinitiation complex assembly [GO:0071163], shelterin complex assembly [GO:0071573], MCM complex loading [GO:0140530], telomere-telomerase complex assembly [GO:1905324]